{
  "gene_name": "Myoblast determination protein 1",
  "gene_symbol": "MYOD1",
  "term_id": "UNKNOWN:0003",
  "term_label": "Unknown cellular component",
  "gene": "UniProtKB:P15172"
}